determination of left/right asymmetry in diencephalon [GO:0035462] (biological process) References: PMID:15084459 Sources: GOC:dgh Definition: The establishment of the diencephalon with respect to the left and right halves. Relationships: is a type of determination of left/right asymmetry in nervous system [GO:0035545]; is part of diencephalon development [GO:0021536]